{
  "gene": "UniProtKB:Q8N8Q8",
  "term_label": "protein insertion into mitochondrial inner membrane from matrix",
  "term_id": "GO:0032979",
  "gene_symbol": "COX18",
  "gene_name": "Cytochrome c oxidase assembly protein COX18, mitochondrial"
}